{
  "gene": "UniProtKB:Q13625",
  "gene_name": "Apoptosis-stimulating of p53 protein 2",
  "term_id": "GO:0002039",
  "term_label": "p53 binding",
  "gene_symbol": "TP53BP2"
}